{
  "gene_name": "Complement C1q subcomponent subunit A",
  "term_label": "Unknown biological process",
  "gene": "UniProtKB:P02745",
  "gene_symbol": "C1QA",
  "term_id": "UNKNOWN:0002"
}